{
  "term_id": "GO:0004571",
  "gene": "UniProtKB:Q9BZQ6",
  "gene_name": "ER degradation-enhancing alpha-mannosidase-like protein 3",
  "gene_symbol": "EDEM3",
  "term_label": "mannosyl-oligosaccharide 1,2-alpha-mannosidase activity"
}